cofilin-actin rod [GO:0090732] (cellular component) Definition: A cellular structure consisting of parallel, hexagonally arranged actin tubules, comprising filamentous actin and disulfide cross-linked cofilin multimers. References: PMID:22573689, PMID:24760020 Sources: GOC:sl Relationships: is a type of actin rod [GO:0031002]